{
  "gene": "UniProtKB:Q13615",
  "term_label": "phosphatidylinositol-3,5-bisphosphate 3-phosphatase activity",
  "gene_name": "Myotubularin-related protein 3",
  "gene_symbol": "MTMR3",
  "term_id": "GO:0052629"
}